{
  "term_id": "GO:0045039",
  "gene_name": "Mitochondrial import inner membrane translocase subunit Tim29",
  "gene_symbol": "TIMM29",
  "term_label": "protein insertion into mitochondrial inner membrane",
  "gene": "UniProtKB:Q9BSF4"
}